{
  "gene": "UniProtKB:P61224",
  "term_label": "negative regulation of synaptic vesicle exocytosis",
  "term_id": "GO:2000301",
  "gene_symbol": "RAP1B",
  "gene_name": "Ras-related protein Rap-1b"
}